thiamine catabolic process [GO:0009230] (biological process) Relationships: is a type of GO:0006772; is a type of primary alcohol catabolic process [GO:0034310]; is a type of GO:0042725 Sources: GOC:jl, ISBN:0198506732 Also known as: thiamin catabolic process, thiamine breakdown, thiamine catabolism, thiamine degradation, vitamin B1 catabolic process, vitamin B1 catabolism Definition: The chemical reactions and pathways resulting in the breakdown of thiamine (vitamin B1), a water soluble vitamin present in fresh vegetables and meats, especially liver.